{
  "term_label": "Unknown biological process",
  "term_id": "UNKNOWN:0002",
  "gene_name": "Immunoglobulin heavy joining 5 (Fragment)",
  "gene_symbol": "IGHJ5",
  "gene": "UniProtKB:A0A0J9YVP9"
}